{
  "term_id": "UNKNOWN:0003",
  "gene_symbol": "THEGL",
  "gene": "UniProtKB:P0DJG4",
  "term_label": "Unknown cellular component",
  "gene_name": "Testicular haploid expressed gene protein-like"
}